copper ion transport across blood-cerebrospinal fluid barrier [GO:0097717] (biological process) Relationships: is a type of copper ion transport [GO:0006825]; is a type of transport across blood-cerebrospinal fluid barrier [GO:0150195] Also known as: copper ion transport across BCSFB, copper ion transport across blood-CSF barrier, copper ion transport across blood/CSF barrier, copper ion transport across blood/cerebrospinal fluid barrier, copper ion transport across BCB References: PMID:24614235 Sources: GOC:sl Definition: The directed movement of copper (Cu) ions passing through the blood-cerebrospinal fluid barrier.